nucleotide catabolic process [GO:0009166] (BP) Relationships: is a type of nucleotide metabolic process [GO:0009117]; is a type of nucleoside phosphate catabolic process [GO:1901292] Also known as: nucleotide breakdown, nucleotide catabolism, nucleotide degradation Sources: GOC:go_curators Regulation: regulated by GO:0030811; negatively regulated by negative regulation of nucleotide catabolic process [GO:0030812]; positively regulated by GO:0030813 Definition: The chemical reactions and pathways resulting in the breakdown of nucleotides, any nucleoside that is esterified with (ortho)phosphate or an oligophosphate at any hydroxyl group on the glycose moiety; may be mono-, di- or triphosphate; this definition includes cyclic-nucleotides (nucleoside cyclic phosphates). Subtypes: purine nucleotide catabolic process [GO:0006195], pyrimidine nucleotide catabolic process [GO:0006244], GO:0009214, ribonucleotide catabolic process [GO:0009261], deoxyribonucleotide catabolic process [GO:0009264], bis(5'-nucleosidyl) oligophosphate catabolic process [GO:0015958], diadenosine polyphosphate catabolic process [GO:0015961], pyridine nucleotide catabolic process [GO:0019364], flavin adenine dinucleotide catabolic process [GO:0072389]